{
  "gene_symbol": "COX7A1",
  "term_id": "GO:0030674",
  "term_label": "protein-macromolecule adaptor activity",
  "gene_name": "Cytochrome c oxidase subunit 7A1, mitochondrial",
  "gene": "UniProtKB:P24310"
}